{
  "gene": "UniProtKB:Q3MIP1",
  "term_id": "UNKNOWN:0001",
  "gene_name": "Inositol 1,4,5-trisphosphate receptor-interacting protein-like 2",
  "gene_symbol": "ITPRIPL2",
  "term_label": "Unknown molecular function"
}